{
  "gene": "UniProtKB:Q9NVP4",
  "term_id": "GO:0042462",
  "term_label": "eye photoreceptor cell development",
  "gene_name": "Double zinc ribbon and ankyrin repeat-containing protein 1",
  "gene_symbol": "DZANK1"
}